secondary metabolic process [GO:0019748] (biological process) Relationships: is a type of metabolic process [GO:0008152] Definition: The chemical reactions and pathways resulting in many of the chemical changes of compounds that are not necessarily required for growth and maintenance of cells, and are often unique to a taxon. In multicellular organisms secondary metabolism is generally carried out in specific cell types, and may be useful for the organism as a whole. In unicellular organisms, secondary metabolism is often used for the production of antibiotics or for the utilization and acquisition of unusual nutrients. Sources: GOC:go_curators Subtypes: melanin metabolic process [GO:0006582], siderophore metabolic process [GO:0009237], toxin metabolic process [GO:0009404], GO:0009698, polyketide metabolic process [GO:0030638], asperthecin metabolic process [GO:0036182], penicillin metabolic process [GO:0042316], GO:0042810, GO:0044550, ocellus pigment metabolic process [GO:0046158], secondary metabolite catabolic process [GO:0090487], diorcinol metabolic process [GO:1900570], violaceol I metabolic process [GO:1900588], violaceol II metabolic process [GO:1900591], GO:1900797, GO:1900813, GO:1900819, GO:1902086 Also known as: secondary metabolism, secondary metabolite metabolic process, secondary metabolite metabolism Regulation: RO_0002211 by regulation of secondary metabolic process [GO:0043455]